maternal aggressive behavior [GO:0002125] (BP) Relationships: is a type of aggressive behavior [GO:0002118] Note: Paternal aggression also exists. Serves to protect the offspring from intruders. Definition: Aggressive behavior of a female to protect her offspring from a threat. Also known as: maternal aggression Sources: GOC:hjd